host-seeking behavior [GO:0032537] (biological process) Definition: The specific behavior of an organism that are associated with finding a host organism; may include behavioral responses to light, temperature, or chemical emanations from the prospective host. Also known as: host-seeking behaviour References: PMID:11931033 Sources: GOC:mah, GOC:pr Relationships: is a type of GO:0007610 Regulation: regulated by regulation of host-seeking behavior [GO:0032538]; negatively regulated by negative regulation of host-seeking behavior [GO:0032539]; positively regulated by positive regulation of host-seeking behavior [GO:0032540]